{
  "gene_symbol": "OAZ3",
  "term_label": "ornithine decarboxylase inhibitor activity",
  "term_id": "GO:0008073",
  "gene_name": "Ornithine decarboxylase antizyme 3",
  "gene": "UniProtKB:Q9UMX2"
}